{
  "term_id": "UNKNOWN:0002",
  "gene_name": "Zinc finger protein 432",
  "gene_symbol": "ZNF432",
  "gene": "UniProtKB:O94892",
  "term_label": "Unknown biological process"
}